{
  "gene_symbol": "OSGIN2",
  "gene_name": "Oxidative stress-induced growth inhibitor 2",
  "term_id": "GO:0008083",
  "gene": "UniProtKB:Q9Y236",
  "term_label": "growth factor activity"
}